{
  "term_id": "GO:0050870",
  "gene": "UniProtKB:P13762",
  "term_label": "positive regulation of T cell activation",
  "gene_name": "HLA class II histocompatibility antigen, DR beta 4 chain",
  "gene_symbol": "HLA-DRB4"
}